pyrimidine nucleobase transmembrane transporter activity [GO:0005350] (molecular function) Subtypes: cytosine transmembrane transporter activity [GO:0015209], GO:0015210, pyrimidine- and adenosine-specific:sodium symporter activity [GO:0015389] Relationships: is a type of nucleobase transmembrane transporter activity [GO:0015205]; is part of pyrimidine nucleobase transport [GO:0015855]; is part of pyrimidine-containing compound transmembrane transport [GO:0072531] Sources: GOC:ai Definition: Enables the transfer of pyrimidine nucleobases, one of the two classes of nitrogen-containing ring compounds found in DNA and RNA, from one side of a membrane to the other. Also known as: pyrimidine base transmembrane transporter activity, pyrimidine transmembrane transporter activity